{
  "gene": "UniProtKB:Q9HCD6",
  "gene_name": "Protein TANC2",
  "gene_symbol": "TANC2",
  "term_label": "regulation of dendritic spine morphogenesis",
  "term_id": "GO:0061001"
}